{
  "gene": "UniProtKB:O00287",
  "gene_symbol": "RFXAP",
  "term_id": "UNKNOWN:0001",
  "term_label": "Unknown molecular function",
  "gene_name": "Regulatory factor X-associated protein"
}